{
  "term_id": "GO:0008076",
  "gene_name": "Leucine-rich repeat-containing protein 55",
  "term_label": "voltage-gated potassium channel complex",
  "gene": "UniProtKB:Q6ZSA7",
  "gene_symbol": "LRRC55"
}